{
  "term_id": "GO:0007399",
  "gene_name": "COUP transcription factor 1",
  "term_label": "nervous system development",
  "gene_symbol": "NR2F1",
  "gene": "UniProtKB:P10589"
}